{
  "gene": "UniProtKB:P55157",
  "gene_name": "Microsomal triglyceride transfer protein large subunit",
  "term_label": "cholesterol homeostasis",
  "gene_symbol": "MTTP",
  "term_id": "GO:0042632"
}